{
  "gene_symbol": "RALGAPA2",
  "term_label": "Unknown biological process",
  "gene": "UniProtKB:Q2PPJ7",
  "gene_name": "Ral GTPase-activating protein subunit alpha-2",
  "term_id": "UNKNOWN:0002"
}